(S)-2-haloacid dehalogenase activity [GO:0018784] (molecular function) Definition: Catalysis of the reaction: (S)-2-haloacid + H2O = (R)-2-hydroxyacid + halide. Sources: EC:3.8.1.2 Relationships: is a type of hydrolase activity, acting on acid halide bonds, in C-halide compounds [GO:0019120] Also known as: 2-haloacid dehalogenase activity, (S)-2-haloacid halidohydrolase activity, 2-haloacid halidohydrolase activity, 2-haloalkanoic acid dehalogenase activity, 2-haloalkanoid acid halidohydrolase activity, 2-halocarboxylic acid dehalogenase II activity, DL-2-haloacid dehalogenase activity, L-2-haloacid dehalogenase activity, L-DEX activity, halocarboxylic acid halidohydrolase activity